{
  "gene": "UniProtKB:O95754",
  "gene_symbol": "SEMA4F",
  "gene_name": "Semaphorin-4F",
  "term_id": "GO:0030335",
  "term_label": "positive regulation of cell migration"
}